{
  "gene_name": "Nuclear pore complex protein Nup98-Nup96",
  "term_label": "protein import into nucleus",
  "gene": "UniProtKB:P52948",
  "gene_symbol": "NUP98",
  "term_id": "GO:0006606"
}